{
  "gene": "UniProtKB:P08620",
  "term_id": "GO:0008543",
  "gene_name": "Fibroblast growth factor 4",
  "gene_symbol": "FGF4",
  "term_label": "fibroblast growth factor receptor signaling pathway"
}